{
  "term_id": "GO:0005634",
  "gene_symbol": "FEV",
  "gene": "UniProtKB:Q99581",
  "term_label": "nucleus",
  "gene_name": "Protein FEV"
}